{
  "term_label": "Unknown biological process",
  "gene": "UniProtKB:Q6PP77",
  "gene_symbol": "XKRX",
  "term_id": "UNKNOWN:0002",
  "gene_name": "XK-related protein 2"
}